estrus [GO:0060209] (biological process) Also known as: oestrus Definition: The estrous cycle phase in which a female is sexually receptive. Sources: GOC:dph, ISBN:0721662544 Relationships: is a type of estrous cycle phase [GO:0060206] Note: Note that this term should not be used for direct annotation. If you are trying to make an annotation to x phase, it is likely that the correct annotation is 'regulation of x/y phase transition' or to a process which occurs during the reported phase. To capture the phase when a specific location or process is observed, the phase term can be used in an annotation extension (PMID:24885854) applied to a cellular component term (with the relation exists_during) or a biological process term (with the relation happens_during).